{
  "gene_name": "Sulfotransferase 4A1",
  "term_id": "GO:0051923",
  "gene": "UniProtKB:Q9BR01",
  "term_label": "sulfation",
  "gene_symbol": "SULT4A1"
}